mesenchymal-epithelial cell signaling involved in prostate induction [GO:0060521] (biological process) Relationships: is a type of inductive mesenchymal to epithelial cell signaling [GO:0060522]; is a type of GO:0060739; is part of prostate induction [GO:0060514] References: PMID:18977204 Sources: GOC:dph Also known as: mesenchymal-epithelial cell signalling involved in prostate induction Definition: Signaling at short range from urogenital sinus mesenchymal cells to cells of the urogenital epithelium resulting in the epithelial cells adopting a prostatic fate.